4-hydroxybenzoate decarboxylase activity [GO:0018799] (molecular function) Definition: Catalysis of the reaction: 4-hydroxybenzoate + H+ = CO2 + phenol. Sources: EC:4.1.1.61, RHEA:10876 Also known as: 4-hydroxybenzoate carboxy-lyase (phenol-forming), 4-hydroxybenzoate carboxy-lyase activity, p-hydroxybenzoate decarboxylase activity Relationships: is a type of carboxy-lyase activity [GO:0016831]